positive regulation of response to G2 DNA damage checkpoint signaling [GO:1902158] (BP) Also known as: activation of G2/M transition DNA damage checkpoint effector process, activation of response to signal involved in G2/M transition DNA damage checkpoint, positive regulation of G2/M transition DNA damage checkpoint effector process, positive regulation of response to signal involved in G2/M transition DNA damage checkpoint, up regulation of G2/M transition DNA damage checkpoint effector process, up regulation of response to G2 DNA damage checkpoint signaling, up regulation of response to signal involved in G2/M transition DNA damage checkpoint, up-regulation of G2/M transition DNA damage checkpoint effector process, up-regulation of response to G2 DNA damage checkpoint signaling, up-regulation of response to signal involved in G2/M transition DNA damage checkpoint, upregulation of G2/M transition DNA damage checkpoint effector process, upregulation of response to G2 DNA damage checkpoint signaling, upregulation of response to signal involved in G2/M transition DNA damage checkpoint, activation of response to G2 DNA damage checkpoint signaling Relationships: is a type of positive regulation of response to DNA damage checkpoint signaling [GO:1902154]; is a type of regulation of response to G2 DNA damage checkpoint signaling [GO:1902157]; positively regulates response to G2 DNA damage checkpoint signaling [GO:0072426] Sources: GOC:TermGenie, GOC:mtg_cell_cycle Definition: Any process that activates or increases the frequency, rate or extent of response to G2 DNA damage checkpoint signaling.